{
  "gene_name": "Uncharacterized protein C20orf144",
  "term_id": "UNKNOWN:0003",
  "gene": "UniProtKB:Q9BQM9",
  "gene_symbol": "C20orf144",
  "term_label": "Unknown cellular component"
}